{
  "term_label": "Unknown molecular function",
  "gene": "UniProtKB:P0DJI9",
  "gene_name": "Serum amyloid A-2 protein",
  "gene_symbol": "SAA2",
  "term_id": "UNKNOWN:0001"
}